{
  "term_label": "Unknown molecular function",
  "gene_symbol": "C2CD4A",
  "gene": "UniProtKB:Q8NCU7",
  "gene_name": "C2 calcium-dependent domain-containing protein 4A",
  "term_id": "UNKNOWN:0001"
}